{
  "term_label": "endoplasmic reticulum",
  "gene_name": "Ankyrin repeat and LEM domain-containing protein 2",
  "gene": "UniProtKB:Q86XL3",
  "term_id": "GO:0005783",
  "gene_symbol": "ANKLE2"
}